{
  "gene_name": "FYVE, RhoGEF and PH domain-containing protein 1",
  "term_label": "guanyl-nucleotide exchange factor activity",
  "term_id": "GO:0005085",
  "gene_symbol": "FGD1",
  "gene": "UniProtKB:P98174"
}